{
  "gene": "UniProtKB:Q50LG9",
  "term_id": "GO:0038023",
  "gene_name": "Leucine-rich repeat-containing protein 24",
  "gene_symbol": "LRRC24",
  "term_label": "signaling receptor activity"
}